{
  "term_label": "Unknown molecular function",
  "gene": "UniProtKB:Q969W3",
  "gene_name": "Protein FAM104A",
  "term_id": "UNKNOWN:0001",
  "gene_symbol": "FAM104A"
}